siRNA-independent facultative heterochromatin formation [GO:1902794] (biological process) References: PMID:22144463, PMID:24210919 Also known as: heterochromatin island assembly, heterochromatin island formation, siRNA-independent facultative heterochromatin assembly Definition: The formation of facultative heterochromatin into a heterochromatin domain, enriched in histone H3 methylated on lysine 9 (H3K9me), by a process independent of small interfering RNAs. Regulation: regulated by regulation of siRNA-independent facultative heterochromatin formation [GO:1902801] Relationships: is a type of facultative heterochromatin formation [GO:0140718]